{
  "term_label": "axon terminus",
  "term_id": "GO:0043679",
  "gene_symbol": "SNCG",
  "gene_name": "Gamma-synuclein",
  "gene": "UniProtKB:O76070"
}